phosphatidylserine floppase activity [GO:0090556] (molecular function) References: PMID:16452632, PMID:20224745 Sources: GOC:ab, RHEA:38567 Also known as: ATPase-coupled phosphatidylserine transporter activity, ATPase-dependent phosphatidylserine transporter activity, phosphatidylserine-translocating ATPase activity, phosphatidylserine floppase activity (cytosolic to exoplasmic leaflet) Definition: Catalysis of the movement of phosphatidylserine from the cytosolic to the exoplasmic leaflet of a membrane, using energy from the hydrolysis of ATP. Relationships: is a type of phospholipid transporter activity [GO:0005548]; is a type of floppase activity [GO:0140328]